{
  "gene_name": "Ewing's tumor-associated antigen 1",
  "gene_symbol": "ETAA1",
  "gene": "UniProtKB:Q9NY74",
  "term_id": "GO:0043596",
  "term_label": "nuclear replication fork"
}